{
  "gene_name": "Putative metallothionein MT1DP",
  "gene": "UniProtKB:A1L3X4",
  "term_label": "detoxification of copper ion",
  "gene_symbol": "MT1DP",
  "term_id": "GO:0010273"
}